p-cymene methyl hydroxylase activity [GO:0018694] (molecular function) Sources: RHEA:51604 Definition: Catalysis of the reaction: 2 H+ + O2 + p-cymene + 2 reduced [2Fe-2S]-[ferredoxin] = 4-isopropylbenzyl alcohol + H2O + 2 oxidized [2Fe-2S]-[ferredoxin]. Relationships: is a type of oxidoreductase activity, acting on paired donors, with incorporation or reduction of molecular oxygen, reduced iron-sulfur protein as one donor, and incorporation of one atom of oxygen [GO:0016713]